{
  "term_label": "negative regulation of ERK1 and ERK2 cascade",
  "gene_symbol": "SPRY3",
  "term_id": "GO:0070373",
  "gene_name": "Protein sprouty homolog 3",
  "gene": "UniProtKB:O43610"
}